{
  "gene_name": "Magnesium transporter MRS2 homolog, mitochondrial",
  "term_id": "GO:0015095",
  "term_label": "magnesium ion transmembrane transporter activity",
  "gene": "UniProtKB:Q9HD23",
  "gene_symbol": "MRS2"
}